{
  "gene": "UniProtKB:Q9UPY8",
  "term_label": "microtubule plus-end binding",
  "term_id": "GO:0051010",
  "gene_name": "Microtubule-associated protein RP_EB family member 3",
  "gene_symbol": "MAPRE3"
}